p-aminobenzoyl-glutamate transmembrane transport [GO:1902604] (biological process) Relationships: is a type of p-aminobenzoyl-glutamate transport [GO:0015814]; is a type of dipeptide transmembrane transport [GO:0035442]; is a type of GO:1905039 Also known as: N-(4-aminobenzoyl)-L-glutamate transmembrane transport Definition: The directed movement of N-(4-aminobenzoyl)-L-glutamate across a membrane. Sources: GOC:TermGenie, GOC:pr, GO_REF:0000069